{
  "term_label": "N-acetylglucosamine catabolic process",
  "gene_symbol": "GNPDA2",
  "gene_name": "Glucosamine-6-phosphate isomerase 2",
  "gene": "UniProtKB:Q8TDQ7",
  "term_id": "GO:0006046"
}